{
  "gene_name": "Coiled-coil domain-containing protein 113",
  "gene": "UniProtKB:Q9H0I3",
  "gene_symbol": "CCDC113",
  "term_label": "cilium assembly",
  "term_id": "GO:0060271"
}